{
  "gene_symbol": "GGT6",
  "term_label": "Unknown biological process",
  "term_id": "UNKNOWN:0002",
  "gene_name": "Glutathione hydrolase 6",
  "gene": "UniProtKB:Q6P531"
}